{
  "term_label": "cAMP-dependent protein kinase complex",
  "gene": "UniProtKB:P51817",
  "gene_name": "cAMP-dependent protein kinase catalytic subunit PRKX",
  "gene_symbol": "PRKX",
  "term_id": "GO:0005952"
}